quercetin-3,3'-bissulfate 7-sulfotransferase activity [GO:0047367] (molecular function) Also known as: quercetin-3,3'-bissulphate 7-sulphotransferase activity, 3'-phosphoadenylyl-sulfate:quercetin-3,3'-bissulfate 7-sulfotransferase activity, 7-sulfotransferase activity, PAPS:flavonol 3,3'/3,4'-disulfate 7-sulfotransferase activity, flavonol 7-sulfotransferase activity Sources: EC:2.8.2.28, MetaCyc:2.8.2.28-RXN Definition: Catalysis of the reaction: quercetin 3,3'-bissulfate + 3'-phosphoadenosine 5'-phosphosulfate = quercetin 3,3',7-trissulfate + adenosine 3',5'-bisphosphate. Relationships: is a type of GO:0008146